{
  "gene_symbol": "CSH2",
  "gene": "UniProtKB:P0DML3",
  "term_id": "GO:0060396",
  "gene_name": "Chorionic somatomammotropin hormone 2",
  "term_label": "growth hormone receptor signaling pathway"
}